{
  "term_id": "GO:0061631",
  "gene": "UniProtKB:Q96LR5",
  "term_label": "ubiquitin conjugating enzyme activity",
  "gene_symbol": "UBE2E2",
  "gene_name": "Ubiquitin-conjugating enzyme E2 E2"
}